{
  "term_id": "GO:0005739",
  "term_label": "mitochondrion",
  "gene_symbol": "TMEM143",
  "gene": "UniProtKB:Q96AN5",
  "gene_name": "Transmembrane protein 143"
}